{
  "gene": "UniProtKB:P52630",
  "gene_name": "Signal transducer and activator of transcription 2",
  "gene_symbol": "STAT2",
  "term_id": "GO:0007259",
  "term_label": "cell surface receptor signaling pathway via JAK-STAT"
}